{
  "gene_symbol": "PSG2",
  "term_id": "GO:0007157",
  "gene_name": "Pregnancy-specific beta-1-glycoprotein 2",
  "gene": "UniProtKB:P11465",
  "term_label": "heterophilic cell-cell adhesion"
}